{
  "term_id": "GO:0044027",
  "gene_name": "Lymphoid-specific helicase",
  "term_label": "negative regulation of gene expression via chromosomal CpG island methylation",
  "gene": "UniProtKB:Q9NRZ9",
  "gene_symbol": "HELLS"
}